bile acid nuclear receptor activity [GO:0038186] (molecular function) Definition: A nuclear receptor activity regulated by a bile acid binding and modulating the transcription of specific gene sets transcribed by RNA polymerase II. References: PMID:32480317, PMID:35415765, PMID:36409000 Relationships: is a type of nuclear receptor activity [GO:0004879]; has part bile acid binding [GO:0032052] Also known as: lithocholic acid receptor activity, farnesoid X nuclear receptor activity, farnesoid X receptor activity